{
  "term_label": "Unknown molecular function",
  "gene": "UniProtKB:Q86X59",
  "gene_symbol": "LINC02875",
  "gene_name": "Putative uncharacterized protein LINC02875",
  "term_id": "UNKNOWN:0001"
}